regulation of brassinosteroid mediated signaling pathway [GO:1900457] (biological process) Definition: Any process that modulates the frequency, rate or extent of brassinosteroid mediated signaling pathway. References: PMID:21855796 Sources: GOC:TermGenie Also known as: regulation of brassinosteroid mediated signalling Relationships: is a type of regulation of signal transduction [GO:0009966]; regulates brassinosteroid mediated signaling pathway [GO:0009742] Subtypes: negative regulation of brassinosteroid mediated signaling pathway [GO:1900458], positive regulation of brassinosteroid mediated signaling pathway [GO:1900459]